{
  "term_id": "GO:0035299",
  "term_label": "inositol-1,3,4,5,6-pentakisphosphate 2-kinase activity",
  "gene": "UniProtKB:Q9H8X2",
  "gene_name": "Inositol-pentakisphosphate 2-kinase",
  "gene_symbol": "IPPK"
}